{
  "gene": "UniProtKB:Q96C01",
  "term_id": "GO:0005737",
  "gene_name": "Protein FAM136A",
  "term_label": "cytoplasm",
  "gene_symbol": "FAM136A"
}